positive regulation of heparan sulfate proteoglycan biosynthetic process [GO:0010909] (biological process) Relationships: is a type of GO:0010908; is a type of positive regulation of proteoglycan biosynthetic process [GO:1902730]; is a type of positive regulation of protein O-linked glycosylation [GO:1904100]; positively regulates heparan sulfate proteoglycan biosynthetic process [GO:0015012] Sources: GOC:curators Definition: Any process that increases the rate, frequency or extent of heparan sulfate proteoglycan biosynthesis. Heparan sulfate proteoglycan biosynthetic processes are the chemical reactions and pathways resulting in the formation of the heparan sulfate proteoglycan, which consists of a core protein linked to a heparan sulfate glycosaminoglycan. The heparan sulfate chain is composed of the repeating disaccharide unit beta-(1,4)-N-acetyl-D-glucosamine-alpha-(1,4)-hexuronic acid.